regulation of very-low-density lipoprotein particle remodeling [GO:0010901] (biological process) Relationships: is a type of regulation of cellular component organization [GO:0051128]; is a type of GO:0051239; regulates GO:0034372 Also known as: regulation of VLDL remodeling, regulation of VLDL remodelling, regulation of very-low-density lipoprotein particle remodelling Sources: GOC:tb Definition: Any process that modulates the rate, frequency or extent of very-low-density lipoprotein particle remodeling. Very-low-density lipoprotein particle remodeling is the acquisition, loss or modification of a protein or lipid within a very-low-density lipoprotein particle, including the hydrolysis of triglyceride by hepatic lipase or lipoprotein lipase and the subsequent loss of free fatty acid. Subtypes: positive regulation of very-low-density lipoprotein particle remodeling [GO:0010902], GO:0010903